{
  "term_label": "Unknown cellular component",
  "term_id": "UNKNOWN:0003",
  "gene_symbol": "SPEM2",
  "gene_name": "Uncharacterized protein SPEM2",
  "gene": "UniProtKB:Q0P670"
}